apical proximal dendrite [GO:0150015] (cellular component) References: PMID:16899232, PMID:1720142, PMID:9214543 Sources: GOC:aruk, GOC:bc Relationships: is_a apical dendrite [GO:0097440]; is a type of GO:1990635 Definition: The dendrite of the dendritic tree, which emerges near the apical pole of a neuron, and which is the closest to the cell body of the neuron (the soma).